{
  "term_id": "GO:0031852",
  "gene_symbol": "GNAO1",
  "term_label": "mu-type opioid receptor binding",
  "gene": "UniProtKB:P09471",
  "gene_name": "Guanine nucleotide-binding protein G(o) subunit alpha"
}